{
  "term_id": "GO:0005634",
  "term_label": "nucleus",
  "gene": "UniProtKB:C9JCN9",
  "gene_name": "Heat shock factor-binding protein 1-like protein 1",
  "gene_symbol": "HSBP1L1"
}